{
  "gene": "UniProtKB:Q9NQ75",
  "gene_symbol": "CASS4",
  "term_id": "GO:0005737",
  "term_label": "cytoplasm",
  "gene_name": "Cas scaffolding protein family member 4"
}